{
  "gene_name": "Exportin-6",
  "term_label": "protein export from nucleus",
  "term_id": "GO:0006611",
  "gene_symbol": "XPO6",
  "gene": "UniProtKB:Q96QU8"
}